{
  "term_label": "chromatin",
  "gene_symbol": "TCF4",
  "term_id": "GO:0000785",
  "gene_name": "Transcription factor 4",
  "gene": "UniProtKB:P15884"
}